{
  "term_id": "UNKNOWN:0001",
  "gene": "UniProtKB:Q8WUY1",
  "gene_name": "Protein THEM6",
  "gene_symbol": "THEM6",
  "term_label": "Unknown molecular function"
}